negative regulation of lymphotoxin A production [GO:0032721] (biological process) Definition: Any process that stops, prevents, or reduces the frequency, rate, or extent of lymphotoxin A production. Sources: GOC:mah Also known as: down regulation of lymphotoxin A production, down-regulation of lymphotoxin A production, downregulation of lymphotoxin A production, negative regulation of LTA production, negative regulation of TNF-beta production, negative regulation of lymphotoxin-alpha production, negative regulation of tumor necrosis factor-beta production, inhibition of lymphotoxin A production, negative regulation of lymphotoxin A biosynthetic process Relationships: is a type of regulation of lymphotoxin A production [GO:0032681]; is_a negative regulation of protein metabolic process [GO:0051248]; is a type of GO:1903556; negatively regulates lymphotoxin A production [GO:0032641]